{
  "gene": "UniProtKB:Q8IWU6",
  "term_id": "GO:0040037",
  "gene_symbol": "SULF1",
  "gene_name": "Extracellular sulfatase Sulf-1",
  "term_label": "negative regulation of fibroblast growth factor receptor signaling pathway"
}